{
  "gene_name": "Killer cell immunoglobulin-like receptor 2DL2",
  "term_id": "GO:0004888",
  "term_label": "transmembrane signaling receptor activity",
  "gene": "UniProtKB:P43627",
  "gene_symbol": "KIR2DL2"
}